feminization of hermaphrodite soma [GO:0042004] (biological process) Sources: GOC:ems Definition: Promotion of female sex and sexual phenotypes in the hermaphroditic soma. An example of this is found in Caenorhabditis elegans. Relationships: is a type of hermaphrodite somatic sex determination [GO:0042001]